{
  "gene": "UniProtKB:Q14061",
  "term_label": "copper chaperone activity",
  "term_id": "GO:0016531",
  "gene_name": "Cytochrome c oxidase copper chaperone",
  "gene_symbol": "COX17"
}